{
  "gene_symbol": "FAM25G",
  "gene_name": "Protein FAM25G",
  "gene": "UniProtKB:B3EWG6",
  "term_label": "Unknown cellular component",
  "term_id": "UNKNOWN:0003"
}